{
  "gene": "UniProtKB:Q9UNK4",
  "term_label": "negative regulation of T cell proliferation",
  "gene_symbol": "PLA2G2D",
  "gene_name": "Group IID secretory phospholipase A2",
  "term_id": "GO:0042130"
}